mono-olein transacylation activity [GO:0051264] (molecular function) Relationships: is a type of acylglycerol O-acyltransferase activity [GO:0016411] References: PMID:15364929 Sources: GOC:ai Definition: Catalysis of the reaction: mono-olein + mono-olein = diolein + glycerol. Mono-olein, also known as mono-oleoylglycerol, is the monoglyceride formed from oleic acid, 9-octodecenoic acid; diolein is also known as dioleoylglycerol. Also known as: MOG transacylation, acyl-CoA-independent mono-olein transacylation, mono-oleoylglycerol O-acyltransferase activity, mono-oleoylglycerol transacylase activity, monoolein transacylation, monooleoylglycerol O-acyltransferase activity, monooleoylglycerol transacylase activity